{
  "term_id": "GO:0051963",
  "gene": "UniProtKB:Q7Z6B7",
  "gene_name": "SLIT-ROBO Rho GTPase-activating protein 1",
  "term_label": "regulation of synapse assembly",
  "gene_symbol": "SRGAP1"
}